{
  "term_label": "branched-chain-amino-acid transaminase activity",
  "gene_symbol": "BCAT2",
  "gene_name": "Branched-chain-amino-acid aminotransferase, mitochondrial",
  "gene": "UniProtKB:O15382",
  "term_id": "GO:0004084"
}